detoxification of inorganic compound [GO:0061687] (biological process) Subtypes: detoxification of copper ion [GO:0010273], detoxification of cobalt ion [GO:0010299], GO:0010312, detoxification of mercury ion [GO:0050787], detoxification of hydrogen peroxide [GO:0061691], GO:0071585, cellular detoxification of fluoride [GO:0140114], cellular detoxification of metal ion [GO:0140961], detoxification of aluminum ion [GO:0140982], detoxification of sulfite [GO:0160245], detoxification of iron ion [GO:1990461] Definition: Any process that reduces or removes the toxicity of inorganic compounds. These include transport of such compounds away from sensitive areas and to compartments or complexes whose purpose is sequestration of inorganic compounds. Sources: GOC:vw Relationships: is a type of GO:0098754